{
  "term_id": "UNKNOWN:0001",
  "gene_name": "Embryonic testis differentiation protein homolog A",
  "term_label": "Unknown molecular function",
  "gene_symbol": "ETDA",
  "gene": "UniProtKB:Q3ZM63"
}